{
  "gene_name": "DNA repair protein XRCC3",
  "gene_symbol": "XRCC3",
  "gene": "UniProtKB:O43542",
  "term_label": "telomere maintenance via recombination",
  "term_id": "GO:0000722"
}